{
  "term_label": "Unknown biological process",
  "gene": "UniProtKB:Q8IZS8",
  "term_id": "UNKNOWN:0002",
  "gene_symbol": "CACNA2D3",
  "gene_name": "Voltage-dependent calcium channel subunit alpha-2_delta-3"
}